{
  "gene_name": "Rho guanine nucleotide exchange factor 19",
  "gene_symbol": "ARHGEF19",
  "gene": "UniProtKB:Q8IW93",
  "term_label": "regulation of actin cytoskeleton organization",
  "term_id": "GO:0032956"
}